{
  "gene_symbol": "NECTIN4",
  "gene_name": "Nectin-4",
  "term_label": "homophilic cell-cell adhesion",
  "term_id": "GO:0007156",
  "gene": "UniProtKB:Q96NY8"
}